{
  "gene_symbol": "CNTNAP3B",
  "term_label": "synapse",
  "term_id": "GO:0045202",
  "gene_name": "Contactin-associated protein-like 3B",
  "gene": "UniProtKB:Q96NU0"
}